{
  "term_id": "GO:0006298",
  "gene": "UniProtKB:Q01831",
  "gene_name": "DNA repair protein complementing XP-C cells",
  "gene_symbol": "XPC",
  "term_label": "mismatch repair"
}